negative regulation of biosynthetic process [GO:0009890] (biological process) Definition: Any process that stops, prevents, or reduces the rate of the chemical reactions and pathways resulting in the formation of substances. Sources: GOC:go_curators Also known as: down regulation of biosynthetic process, down-regulation of biosynthetic process, downregulation of biosynthetic process, negative regulation of anabolism, negative regulation of biosynthesis, negative regulation of formation, negative regulation of synthesis, inhibition of biosynthetic process Subtypes: negative regulation of flavonoid biosynthetic process [GO:0009964], negative regulation of macromolecule biosynthetic process [GO:0010558], GO:0030809, GO:0032353, negative regulation of collagen biosynthetic process [GO:0032966], negative regulation of nitric oxide biosynthetic process [GO:0045019], negative regulation of gluconeogenesis [GO:0045721], GO:0051055, negative regulation of thiamine diphosphate biosynthetic process [GO:0070617], negative regulation of reductive pentose-phosphate cycle [GO:0080153], negative regulation of (R)-mevalonic acid biosynthetic process [GO:0106108], negative regulation of UDP-N-acetylglucosamine biosynthetic process [GO:0106279], negative regulation of pyruvate decarboxylation to acetyl-CoA [GO:0160218], negative regulation of polyamine biosynthetic process [GO:0170066], negative regulation of raffinose biosynthetic process [GO:1900092], negative regulation of xanthone-containing compound biosynthetic process [GO:1900184], negative regulation of methanofuran biosynthetic process [GO:1900352], negative regulation of secondary metabolite biosynthetic process [GO:1900377], GO:1900641, GO:1900847, negative regulation of pseurotin A biosynthetic process [GO:1900850], negative regulation of hexadecanal biosynthetic process [GO:1900903], negative regulation of olefin biosynthetic process [GO:1900912], GO:1900963, negative regulation of sarcinapterin biosynthetic process [GO:1900972], negative regulation of tatiopterin biosynthetic process [GO:1900975], negative regulation of phenazine biosynthetic process [GO:1900981], GO:1901464, GO:1901578, negative regulation of fumagillin biosynthetic process [GO:1902091], negative regulation of alcohol biosynthetic process [GO:1902931], negative regulation of dopamine biosynthetic process [GO:1903180], negative regulation of reactive oxygen species biosynthetic process [GO:1903427], negative regulation of lactose biosynthetic process [GO:1903535], negative regulation of glutathione biosynthetic process [GO:1903787], negative regulation of ubiquinone biosynthetic process [GO:1904774], negative regulation of hydrogen sulfide biosynthetic process [GO:1904827], negative regulation of quinolinate biosynthetic process [GO:1904985], negative regulation of serotonin biosynthetic process [GO:1905628], negative regulation of trypanothione biosynthetic process [GO:1905723], GO:1905922, negative regulation of L-ascorbic acid biosynthetic process [GO:2000083], negative regulation of amino acid biosynthetic process [GO:2000283] Relationships: is a type of regulation of biosynthetic process [GO:0009889]; is a type of negative regulation of metabolic process [GO:0009892]; negatively regulates biosynthetic process [GO:0009058]